21U-RNA binding [GO:0034583] (molecular function) Sources: GOC:kmv Definition: Binding to a 21U-RNA, a 21-nucleotide RNA characterized by a uridine 5'-monophosphate and a modified 3' end resistant to periodate degradation. 21U-RNAs are derived from distinct, autonomously expressed loci within the genome. Relationships: is a type of RNA binding [GO:0003723]